{
  "gene": "UniProtKB:Q8NGL4",
  "term_label": "olfactory receptor activity",
  "term_id": "GO:0004984",
  "gene_symbol": "OR5D13",
  "gene_name": "Olfactory receptor 5D13"
}